{
  "gene": "UniProtKB:P60893",
  "term_label": "plasma membrane",
  "term_id": "GO:0005886",
  "gene_name": "Probable G-protein coupled receptor 85",
  "gene_symbol": "GPR85"
}